unmethylated CpG binding [GO:0045322] (molecular function) References: PMID:10688657 Sources: GOC:ai Definition: Binding to uan nmethylated CpG motif. Unmethylated CpG dinucleotides are often associated with gene promoters. Relationships: is a type of sequence-specific DNA binding [GO:0043565]